{
  "gene_symbol": "ABCA5",
  "term_id": "GO:0005319",
  "gene": "UniProtKB:Q8WWZ7",
  "term_label": "lipid transporter activity",
  "gene_name": "Cholesterol transporter ABCA5"
}